{
  "gene": "UniProtKB:Q7Z3V4",
  "term_label": "ubiquitin-dependent protein catabolic process",
  "gene_name": "Ubiquitin-protein ligase E3B",
  "term_id": "GO:0006511",
  "gene_symbol": "UBE3B"
}